acetolactate synthase regulator activity [GO:1990610] (molecular function) Relationships: is a type of GO:0030234; regulates acetolactate synthase activity [GO:0003984] Definition: Binds to and modulates the activity of acetolactate synthase. References: PMID:8972574